filamentous growth of a population of unicellular organisms in response to biotic stimulus [GO:0036180] (biological process) Regulation: regulated by GO:1900443; RO_0002212 by negative regulation of filamentous growth of a population of unicellular organisms in response to biotic stimulus [GO:1900444]; positively regulated by GO:1900445 Relationships: is_a response to biotic stimulus [GO:0009607]; is a type of filamentous growth of a population of unicellular organisms [GO:0044182] Definition: The process in which a group of unicellular organisms grow in a threadlike, filamentous shape in response to a biotic (living) stimulus. Subtypes: GO:0097317 Sources: GOC:di